{
  "term_id": "GO:0003779",
  "gene_name": "Microtubule-associated protein 1S",
  "gene": "UniProtKB:Q66K74",
  "term_label": "actin binding",
  "gene_symbol": "MAP1S"
}